{
  "term_label": "snRNA-activating protein complex",
  "term_id": "GO:0019185",
  "gene_symbol": "SNAPC3",
  "gene": "UniProtKB:Q92966",
  "gene_name": "snRNA-activating protein complex subunit 3"
}